{
  "term_label": "tubulin-glutamic acid ligase activity",
  "gene": "UniProtKB:Q3SXZ7",
  "gene_name": "Probable tubulin polyglutamylase TTLL9",
  "gene_symbol": "TTLL9",
  "term_id": "GO:0070740"
}